nitronate monooxygenase (FMN-linked) activity [GO:0036434] (MF) Definition: Catalysis of the reaction: ethylnitronate + FMNH(2) + O2 = acetaldehyde + FMN + H2O + H+ + nitrite. Sources: RHEA:26458 Relationships: is a type of oxidoreductase activity, acting on single donors with incorporation of molecular oxygen, incorporation of one atom of oxygen (internal monooxygenases or internal mixed function oxidases) [GO:0016703]